{
  "gene_name": "Pseudouridine-5'-phosphatase",
  "gene_symbol": "PUDP",
  "term_id": "UNKNOWN:0003",
  "gene": "UniProtKB:Q08623",
  "term_label": "Unknown cellular component"
}